Golgi inheritance [GO:0048313] (biological process) References: PMID:12851069 Sources: GOC:jid Regulation: regulated by regulation of Golgi inheritance [GO:0090170] Also known as: Golgi apparatus inheritance, Golgi division, Golgi partitioning Definition: The partitioning of Golgi apparatus between daughter cells at cell division. Relationships: is a type of Golgi organization [GO:0007030]; is a type of GO:0048308